glutamyl-tRNA(Gln) amidotransferase complex [GO:0030956] (cellular component) Definition: A protein complex that possesses glutamyl-tRNA(Gln) amidotransferase activity, and therefore creates Gln-tRNA by amidating Glu-tRNA; usually composed of 3 subunits: A, B, and C. Note that the C subunit may not be required in all organisms. Sources: GOC:mlg Also known as: GatCAB, GatFAB, AdT Note: Note that this term represents a location and not a function; the activity possessed by this complex is mentioned in the definition for the purpose of describing and distinguishing the complex. The function possessed by this complex is represented by the molecular function term 'glutaminyl-tRNA synthase (glutamine-hydrolyzing) activity ; GO:0050567'. Relationships: is_a intracellular protein-containing complex [GO:0140535]; is a type of catalytic complex [GO:1902494]